{
  "term_id": "GO:0001669",
  "gene_symbol": "LYZL6",
  "gene_name": "Lysozyme-like protein 6",
  "gene": "UniProtKB:O75951",
  "term_label": "acrosomal vesicle"
}